{
  "gene_name": "EH domain-containing protein 2",
  "gene_symbol": "EHD2",
  "gene": "UniProtKB:Q9NZN4",
  "term_id": "GO:0060271",
  "term_label": "cilium assembly"
}